{
  "gene_symbol": "FANCM",
  "gene_name": "Fanconi anemia group M protein",
  "term_id": "GO:0000400",
  "term_label": "four-way junction DNA binding",
  "gene": "UniProtKB:Q8IYD8"
}